{
  "gene": "UniProtKB:P55735",
  "term_id": "GO:0005198",
  "gene_symbol": "SEC13",
  "gene_name": "Protein SEC13 homolog",
  "term_label": "structural molecule activity"
}